{
  "gene_name": "Spectrin beta chain, erythrocytic",
  "gene_symbol": "SPTB",
  "gene": "UniProtKB:P11277",
  "term_id": "GO:0005886",
  "term_label": "plasma membrane"
}